{
  "gene_symbol": "SHISA2",
  "term_id": "GO:0030178",
  "term_label": "negative regulation of Wnt signaling pathway",
  "gene": "UniProtKB:Q6UWI4",
  "gene_name": "Protein shisa-2 homolog"
}